{
  "term_id": "GO:0030897",
  "gene_symbol": "VPS18",
  "term_label": "HOPS complex",
  "gene": "UniProtKB:Q9P253",
  "gene_name": "Vacuolar protein sorting-associated protein 18 homolog"
}